{
  "term_id": "GO:0035325",
  "gene": "UniProtKB:Q99836",
  "term_label": "Toll-like receptor binding",
  "gene_symbol": "MYD88",
  "gene_name": "Myeloid differentiation primary response protein MyD88"
}